mannitol dehydrogenase (cytochrome) activity [GO:0050087] (molecular function) Definition: Catalysis of the reaction: 2 [Fe(III)cytochrome c] + D-mannitol = 2 [Fe(II)cytochrome c] + D-fructose + 2 H+. Sources: RHEA:17597 Also known as: polyol dehydrogenase activity, D-mannitol:ferricytochrome-c 2-oxidoreductase activity Relationships: is a type of oxidoreductase activity, acting on the CH-OH group of donors, cytochrome as acceptor [GO:0016898]